{
  "gene_name": "Protein mono-ADP-ribosyltransferase PARP15",
  "gene": "UniProtKB:Q460N3",
  "term_id": "GO:0003714",
  "gene_symbol": "PARP15",
  "term_label": "transcription corepressor activity"
}